{
  "gene": "UniProtKB:Q99954",
  "term_id": "GO:0051930",
  "gene_name": "Submaxillary gland androgen-regulated protein 3A",
  "term_label": "regulation of sensory perception of pain",
  "gene_symbol": "SMR3A"
}